{
  "gene_name": "Purine nucleoside phosphorylase LACC1",
  "term_label": "copper ion binding",
  "gene": "UniProtKB:Q8IV20",
  "term_id": "GO:0005507",
  "gene_symbol": "LACC1"
}